{
  "gene_symbol": "ERC2-IT1",
  "gene": "UniProtKB:O76042",
  "term_label": "Unknown biological process",
  "term_id": "UNKNOWN:0002",
  "gene_name": "Putative uncharacterized protein encoded by ERC2-IT1"
}